{
  "term_label": "Unknown molecular function",
  "term_id": "UNKNOWN:0001",
  "gene": "UniProtKB:L0R819",
  "gene_symbol": "ASDURF",
  "gene_name": "ASNSD1 upstream open reading frame protein"
}